{
  "term_id": "UNKNOWN:0003",
  "gene_symbol": "RBPMS",
  "gene": "UniProtKB:Q93062",
  "term_label": "Unknown cellular component",
  "gene_name": "RNA-binding protein with multiple splicing"
}